Fc-gamma receptor I complex [GO:0033000] (cellular component) Relationships: is a type of Fc receptor complex [GO:0032997] Also known as: IgG receptor complex, immunoglobulin G receptor complex, FcgRI complex Definition: A protein complex composed of an Fc-gamma RI alpha chain and an Fc-epsilon RI gamma chain dimer with or without additional signaling components. The complex functions primarily as an activating receptor for IgG. References: PMID:11244038, PMID:12413532 Sources: GOC:add, ISBN:0781735149